{
  "gene": "UniProtKB:Q15760",
  "term_label": "plasma membrane",
  "gene_symbol": "GPR19",
  "gene_name": "Probable G-protein coupled receptor 19",
  "term_id": "GO:0005886"
}